{
  "gene_symbol": "GALNS",
  "gene": "UniProtKB:P34059",
  "term_id": "UNKNOWN:0003",
  "gene_name": "N-acetylgalactosamine-6-sulfatase",
  "term_label": "Unknown cellular component"
}